{
  "term_id": "GO:0005886",
  "term_label": "plasma membrane",
  "gene_name": "Pleckstrin homology domain-containing family A member 1",
  "gene_symbol": "PLEKHA1",
  "gene": "UniProtKB:Q9HB21"
}